{
  "gene_symbol": "FBN2",
  "gene_name": "Fibrillin-2",
  "term_id": "GO:0031012",
  "gene": "UniProtKB:P35556",
  "term_label": "extracellular matrix"
}